{
  "term_id": "GO:0019814",
  "gene_name": "Immunoglobulin kappa variable 1-5",
  "gene_symbol": "IGKV1-5",
  "term_label": "immunoglobulin complex",
  "gene": "UniProtKB:P01602"
}